{
  "gene": "UniProtKB:Q6ZVX7",
  "gene_symbol": "NCCRP1",
  "term_id": "GO:0006516",
  "gene_name": "F-box only protein 50",
  "term_label": "glycoprotein catabolic process"
}